{
  "gene_name": "Cholesterol transporter ABCA5",
  "term_id": "GO:0005770",
  "term_label": "late endosome",
  "gene": "UniProtKB:Q8WWZ7",
  "gene_symbol": "ABCA5"
}